response to nitrogen dioxide [GO:0035713] (biological process) Sources: GOC:BHF Relationships: is_a response to nitrogen compound [GO:1901698]; is a type of response to oxygen-containing compound [GO:1901700] Subtypes: GO:0035714 Definition: Any process that results in a change in state or activity of a cell or an organism (in terms of movement, secretion, enzyme production, gene expression, etc.) as a result of a nitrogen dioxide (NO2) stimulus. Also known as: response to NO2